{
  "term_label": "chemokine-mediated signaling pathway",
  "gene_symbol": "CCL21",
  "gene": "UniProtKB:O00585",
  "term_id": "GO:0070098",
  "gene_name": "C-C motif chemokine 21"
}